{
  "gene_name": "Palmitoyltransferase ZDHHC19",
  "gene": "UniProtKB:Q8WVZ1",
  "term_label": "protein targeting to membrane",
  "gene_symbol": "ZDHHC19",
  "term_id": "GO:0006612"
}